Toll binding [GO:0005121] (molecular function) Sources: GOC:ceb Relationships: is a type of signaling receptor binding [GO:0005102] Also known as: Tl binding, Toll receptor binding, Toll ligand Definition: Binding to a Toll protein, a transmembrane receptor.